positive regulation of apoptosome assembly [GO:1905102] (biological process) Also known as: positive regulation of apoptosome formation, up regulation of apoptosome assembly, up regulation of apoptosome formation, up-regulation of apoptosome assembly, up-regulation of apoptosome formation, upregulation of apoptosome assembly, upregulation of apoptosome formation, activation of apoptosome assembly, activation of apoptosome formation References: PMID:26265044 Sources: GOC:BHF, GOC:BHF_miRNA, GOC:TermGenie, GOC:bc, GO_REF:0000058 Relationships: is a type of positive regulation of protein-containing complex assembly [GO:0031334]; is a type of regulation of apoptosome assembly [GO:1905100]; positively regulates apoptosome assembly [GO:0097314] Definition: Any process that activates or increases the frequency, rate or extent of apoptosome assembly.